1,8-cineole 2-exo-monooxygenase activity [GO:0102320] (molecular function) Definition: Catalysis of the reaction: 1,8-cineole + NADPH + H+ + O2 = 2-exo-hydroxy-1,8-cineole + NADP + H2O. Relationships: is a type of oxidoreductase activity, acting on paired donors, with incorporation or reduction of molecular oxygen, NAD(P)H as one donor, and incorporation of one atom of oxygen [GO:0016709] Sources: GOC:pz, RHEA:32895